{
  "gene_name": "Claudin-17",
  "term_label": "plasma membrane",
  "gene": "UniProtKB:P56750",
  "term_id": "GO:0005886",
  "gene_symbol": "CLDN17"
}